4-chloro-allylglycine synthase activity [GO:0062146] (molecular function) References: PMID:30867596 Sources: RHEA:59888 Relationships: is a type of oxidoreductase activity, acting on paired donors, with incorporation or reduction of molecular oxygen [GO:0016705] Definition: Catalysis of the reaction: 4-chloro-L-lysine + AH2 + O2 = A + formaldehyde + H2O + L-2-amino-4-chloropent-4-enoate + NH4(+).